{
  "term_label": "TBP-class protein binding",
  "gene": "UniProtKB:Q8IZX4",
  "gene_name": "Transcription initiation factor TFIID subunit 1-like",
  "term_id": "GO:0017025",
  "gene_symbol": "TAF1L"
}